larval heart development [GO:0007508] (biological process) Relationships: is a type of heart development [GO:0007507]; is part of larval development [GO:0002164] Definition: The process whose specific outcome is the progression of the larval heart over time, from its formation to the mature structure. In Drosophila the larval heart (dorsal vessel) is a continuous tube of mesodormal cells that runs beneath the dorsal midline of the epidermis, divided into an anterior aorta and a posterior heart proper. Sources: GOC:bf, ISBN:0879694238